{
  "gene_symbol": "CYB5RL",
  "gene": "UniProtKB:Q6IPT4",
  "term_label": "Unknown biological process",
  "gene_name": "NADH-cytochrome b5 reductase-like",
  "term_id": "UNKNOWN:0002"
}